{
  "term_label": "small-subunit processome",
  "gene": "UniProtKB:Q9Y2X3",
  "gene_name": "Nucleolar protein 58",
  "gene_symbol": "NOP58",
  "term_id": "GO:0032040"
}